{
  "gene_symbol": "CTAGE1",
  "term_id": "GO:0009306",
  "gene": "UniProtKB:Q96RT6",
  "term_label": "protein secretion",
  "gene_name": "cTAGE family member 2"
}